{
  "gene": "UniProtKB:Q7Z6M2",
  "term_id": "UNKNOWN:0001",
  "term_label": "Unknown molecular function",
  "gene_symbol": "FBXO33",
  "gene_name": "F-box only protein 33"
}